{
  "gene_name": "Uncharacterized protein C3orf22",
  "term_id": "UNKNOWN:0001",
  "gene": "UniProtKB:Q8N5N4",
  "gene_symbol": "C3orf22",
  "term_label": "Unknown molecular function"
}